{
  "gene": "UniProtKB:Q96SF2",
  "gene_name": "T-complex protein 1 subunit theta-like 2",
  "term_id": "GO:0051082",
  "gene_symbol": "CCT8L2",
  "term_label": "unfolded protein binding"
}